ocellus pigment catabolic process [GO:0046159] (biological process) Also known as: ocellus pigment breakdown, ocellus pigment catabolism, ocellus pigment degradation Definition: The chemical reactions and pathways resulting in the breakdown of ocellus pigments, any general or particular coloring matter in living organisms, found or utilized in the ocellus, a minute simple eye found in many invertebrates. References: PMID:15176085, PMID:18421706 Sources: GOC:ai Relationships: is a type of pigment catabolic process [GO:0046149]; is a type of ocellus pigment metabolic process [GO:0046158] Subtypes: ommochrome catabolic process [GO:0046153]